{
  "gene_name": "Golgi-associated RAB2 interactor protein 3",
  "gene": "UniProtKB:Q8TC56",
  "gene_symbol": "GARIN3",
  "term_label": "Unknown cellular component",
  "term_id": "UNKNOWN:0003"
}